{
  "gene_name": "Izumo sperm-egg fusion protein 3",
  "gene": "UniProtKB:Q5VZ72",
  "term_label": "Unknown molecular function",
  "gene_symbol": "IZUMO3",
  "term_id": "UNKNOWN:0001"
}